{
  "term_label": "melanosome organization",
  "term_id": "GO:0032438",
  "gene_symbol": "PMEL",
  "gene_name": "Melanocyte protein PMEL",
  "gene": "UniProtKB:P40967"
}